{
  "gene": "UniProtKB:Q6UXR8",
  "term_label": "Unknown molecular function",
  "gene_symbol": "UNQ6493_PRO21345",
  "gene_name": "Putative uncharacterized protein UNQ6493_PRO21345",
  "term_id": "UNKNOWN:0001"
}